brain renin-angiotensin system [GO:0002035] (biological process) References: PMID:2909574 Definition: The process in which an angiotensin-mediated signaling system present in the brain regulates the force with which blood passes through the circulatory system. Relationships: is a type of nervous system process involved in regulation of systemic arterial blood pressure [GO:0001976]; is a type of regulation of blood volume by renin-angiotensin [GO:0002016]